{
  "gene": "UniProtKB:A8MVU1",
  "term_id": "GO:0042554",
  "gene_name": "Putative neutrophil cytosol factor 1C",
  "gene_symbol": "NCF1C",
  "term_label": "superoxide anion generation"
}